limonin-D-ring-lactonase activity [GO:0050055] (MF) Sources: EC:3.1.1.36, MetaCyc:LIMONIN-D-RING-LACTONASE-RXN Definition: Catalysis of the reaction: limonoate D-ring-lactone + H2O = limonoate. Also known as: limonin lactone hydrolase activity, limonin-D-ring-lactone hydrolase activity, limonoate-D-ring-lactone lactonohydrolase activity Relationships: is a type of carboxylic ester hydrolase activity [GO:0052689]